regulation of acetylcholine metabolic process [GO:0060408] (biological process) Definition: Any process that modulates the rate, frequency or extent of the chemical reactions and pathways involving acetylcholine, the acetic acid ester of the organic base choline. Acetylcholine is a major neurotransmitter and neuromodulator both in the central and peripheral nervous systems. It also acts as a paracrine signal in various non-neural tissues. Sources: GOC:dph, GOC:tb Relationships: is a type of GO:0033238; is a type of regulation of primary metabolic process [GO:0080090]; regulates acetylcholine metabolic process [GO:0008291] Subtypes: GO:0060409, GO:1905921